{
  "term_label": "insulin-like growth factor II binding",
  "gene_symbol": "IGFBP3",
  "term_id": "GO:0031995",
  "gene": "UniProtKB:P17936",
  "gene_name": "Insulin-like growth factor-binding protein 3"
}